{
  "gene": "UniProtKB:P04080",
  "gene_name": "Cystatin-B",
  "gene_symbol": "CSTB",
  "term_id": "GO:0004869",
  "term_label": "cysteine-type endopeptidase inhibitor activity"
}